{
  "term_id": "GO:0006508",
  "term_label": "proteolysis",
  "gene_name": "Transmembrane gamma-carboxyglutamic acid protein 4",
  "gene": "UniProtKB:Q9BZD6",
  "gene_symbol": "PRRG4"
}